{
  "gene_name": "Alpha-adducin",
  "term_id": "GO:0051015",
  "gene_symbol": "ADD1",
  "term_label": "actin filament binding",
  "gene": "UniProtKB:P35611"
}